{
  "gene_symbol": "CDH4",
  "term_id": "GO:0000902",
  "term_label": "cell morphogenesis",
  "gene": "UniProtKB:P55283",
  "gene_name": "Cadherin-4"
}